2,5-dihydroxypyridine 5,6-dioxygenase activity [GO:0047075] (molecular function) Also known as: 2,5-dihydroxypyridine oxygenase activity, 2,5-dihydroxypyridine:oxygen 5,6-oxidoreductase activity, pyridine-2,5-diol dioxygenase activity Sources: EC:1.13.11.9, MetaCyc:1.13.11.9-RXN Relationships: is a type of GO:0016702 Definition: Catalysis of the reaction: H2O + O2 + 2,5-dihydroxypyridine = formate + maleamate.